{
  "term_label": "calcium ion binding",
  "term_id": "GO:0005509",
  "gene_name": "Calmegin",
  "gene_symbol": "CLGN",
  "gene": "UniProtKB:O14967"
}